{
  "term_label": "membrane",
  "gene": "UniProtKB:Q5VZ19",
  "gene_symbol": "TDRD10",
  "term_id": "GO:0016020",
  "gene_name": "Tudor domain-containing protein 10"
}